{
  "term_label": "basolateral plasma membrane",
  "gene": "UniProtKB:A0A075B734",
  "gene_symbol": "AQP7B",
  "term_id": "GO:0016323",
  "gene_name": "Aquaporin-7B"
}